{
  "term_label": "cytoplasm",
  "gene": "UniProtKB:O00743",
  "term_id": "GO:0005737",
  "gene_name": "Serine_threonine-protein phosphatase 6 catalytic subunit",
  "gene_symbol": "PPP6C"
}